negative regulation of cell proliferation involved in compound eye morphogenesis [GO:2000496] (biological process) Sources: GOC:obol Definition: Any process that stops, prevents or reduces the frequency, rate or extent of cell proliferation involved in compound eye morphogenesis. Relationships: is a type of negative regulation of cell population proliferation [GO:0008285]; is a type of regulation of cell proliferation involved in compound eye morphogenesis [GO:2000495]; negatively regulates GO:0035736